interferon receptor activity [GO:0004904] (molecular function) Definition: Combining with an interferon and transmitting the signal from one side of the membrane to the other to initiate a change in cell activity. Relationships: is a type of cytokine receptor activity [GO:0004896]; has part interferon binding [GO:0019961] References: PMID:9607096 Sources: GOC:ai, GOC:signaling Also known as: IFN receptor activity Subtypes: type I interferon receptor activity [GO:0004905], GO:0004906, GO:0034348